acetyltransferase activator activity [GO:0010698] (MF) References: PMID:23912279 Sources: GOC:dph, GOC:jp, GOC:tb Relationships: is a type of enzyme activator activity [GO:0008047]; positively regulates acetyltransferase activity [GO:0016407] Definition: Binds to and increases the activity of an acetyltransferase, an enzyme which catalyzes the transfer of an acetyl group to an acceptor molecule. Also known as: acetyltransferase stimulator activity